{
  "gene_name": "Codanin-1",
  "term_label": "chromatin organization",
  "gene": "UniProtKB:Q8IWY9",
  "gene_symbol": "CDAN1",
  "term_id": "GO:0006325"
}